{
  "gene": "UniProtKB:Q13347",
  "gene_name": "Eukaryotic translation initiation factor 3 subunit I",
  "term_id": "GO:0071541",
  "gene_symbol": "EIF3I",
  "term_label": "eukaryotic translation initiation factor 3 complex, eIF3m"
}